ascospore wall [GO:0005619] (CC) Definition: The specialized cell wall of the ascospore (spore), which is the product of meiotic division. Examples of this component are found in Fungi. Also known as: fungal-type spore wall Relationships: is a type of fungal-type cell wall [GO:0009277]; is a type of spore wall [GO:0031160] Sources: GOC:vw, ISBN:0879693568